apical protein localization [GO:0045176] (biological process) Definition: Any process in which a protein is transported to, or maintained in, apical regions of the cell. Sources: GOC:bf Also known as: apical protein localisation, establishment and maintenance of apical protein localization, establishment and maintenance of protein localization in apical part of cell Relationships: is a type of intracellular protein localization [GO:0008104]